{
  "gene_name": "Tetraspanin-31",
  "gene": "UniProtKB:Q12999",
  "term_id": "UNKNOWN:0003",
  "term_label": "Unknown cellular component",
  "gene_symbol": "TSPAN31"
}